photoinhibition [GO:0010205] (biological process) Definition: The mechanism by which high light intensity inhibits photosynthesis through inactivation of the D1 protein of photosystem II. Relationships: is a type of response to high light intensity [GO:0009644]; is a type of negative regulation of photosynthesis, light reaction [GO:0043155]; negatively regulates photosynthetic electron transport chain [GO:0009767] Also known as: photosystem II inhibition References: PMID:12068126 Sources: GOC:mtg_electron_transport